{
  "gene": "UniProtKB:Q5VZR2",
  "term_id": "UNKNOWN:0001",
  "gene_name": "NUT family member 2G",
  "term_label": "Unknown molecular function",
  "gene_symbol": "NUTM2G"
}